{
  "term_label": "dystrophin-associated glycoprotein complex",
  "gene_name": "Beta-1-syntrophin",
  "gene_symbol": "SNTB1",
  "gene": "UniProtKB:Q13884",
  "term_id": "GO:0016010"
}